{
  "gene_symbol": "CARM1",
  "gene": "UniProtKB:Q86X55",
  "gene_name": "Histone-arginine methyltransferase CARM1",
  "term_id": "GO:0070611",
  "term_label": "histone H3R2 methyltransferase activity"
}